negative regulation of single strand break repair [GO:1903517] (biological process) Also known as: down regulation of single strand break repair, down-regulation of single strand break repair, downregulation of single strand break repair, inhibition of single strand break repair References: PMID:17395247 Sources: GOC:BHF, GOC:TermGenie, GOC:rl, GO_REF:0000058 Relationships: is a type of negative regulation of DNA repair [GO:0045738]; is a type of regulation of single strand break repair [GO:1903516]; negatively regulates single strand break repair [GO:0000012] Definition: Any process that stops, prevents or reduces the frequency, rate or extent of single strand break repair. Subtypes: negative regulation of single-strand break repair via homologous recombination [GO:1903111], negative regulation of telomere single strand break repair [GO:1903824]